{
  "term_label": "Unknown biological process",
  "gene_symbol": "PNPLA6",
  "term_id": "UNKNOWN:0002",
  "gene_name": "Patatin-like phospholipase domain-containing protein 6",
  "gene": "UniProtKB:Q8IY17"
}